mitotic actomyosin contractile ring, intermediate layer [GO:0120105] (cellular component) References: PMID:28914606 Sources: GOC:krc, GOC:vw Definition: The region of the mitotic actomyosin ring in between the proximal layer and the actin filament layer. This region contains the accessory protein network, some actin filaments and connections between the proximal layer and the actin filament layer. Relationships: is a type of GO:0110165; is part of mitotic actomyosin contractile ring [GO:0110085] Also known as: actomyosin contractile ring, intermediate layer